{
  "term_id": "GO:0001817",
  "gene_name": "Zinc finger and BTB domain-containing protein 12",
  "gene": "UniProtKB:Q9Y330",
  "term_label": "regulation of cytokine production",
  "gene_symbol": "ZBTB12"
}